{
  "gene": "UniProtKB:P61225",
  "term_id": "GO:0005886",
  "gene_symbol": "RAP2B",
  "term_label": "plasma membrane",
  "gene_name": "Ras-related protein Rap-2b"
}